{
  "gene_symbol": "CDNF",
  "term_id": "GO:0031175",
  "term_label": "neuron projection development",
  "gene_name": "Cerebral dopamine neurotrophic factor",
  "gene": "UniProtKB:Q49AH0"
}